{
  "gene": "UniProtKB:Q12794",
  "gene_symbol": "HYAL1",
  "term_label": "cytoplasmic vesicle",
  "term_id": "GO:0031410",
  "gene_name": "Hyaluronidase-1"
}